{
  "term_label": "mitotic G2 DNA damage checkpoint signaling",
  "term_id": "GO:0007095",
  "gene_name": "MRN complex-interacting protein",
  "gene": "UniProtKB:Q6NTE8",
  "gene_symbol": "MRNIP"
}